{
  "gene": "UniProtKB:Q9NS71",
  "term_id": "GO:0005615",
  "gene_symbol": "GKN1",
  "gene_name": "Gastrokine-1",
  "term_label": "extracellular space"
}